{
  "term_label": "double-stranded telomeric DNA binding",
  "term_id": "GO:0003691",
  "gene": "UniProtKB:P54274",
  "gene_name": "Telomeric repeat-binding factor 1",
  "gene_symbol": "TERF1"
}